{
  "gene_symbol": "ESYT2",
  "term_label": "calcium-dependent phospholipid binding",
  "term_id": "GO:0005544",
  "gene": "UniProtKB:A0FGR8",
  "gene_name": "Extended synaptotagmin-2"
}